{
  "gene_name": "Acid sphingomyelinase-like phosphodiesterase 3a",
  "gene": "UniProtKB:Q92484",
  "term_id": "GO:0008081",
  "gene_symbol": "SMPDL3A",
  "term_label": "phosphoric diester hydrolase activity"
}